{
  "gene": "UniProtKB:Q16819",
  "term_id": "GO:0005615",
  "term_label": "extracellular space",
  "gene_name": "Meprin A subunit alpha",
  "gene_symbol": "MEP1A"
}